{
  "gene_name": "Matrin-3",
  "term_label": "nucleus",
  "term_id": "GO:0005634",
  "gene": "UniProtKB:P43243",
  "gene_symbol": "MATR3"
}